{
  "gene_name": "Transcription factor BTF3 homolog 4",
  "gene": "UniProtKB:Q96K17",
  "term_label": "Unknown molecular function",
  "gene_symbol": "BTF3L4",
  "term_id": "UNKNOWN:0001"
}